{
  "term_label": "RNA polymerase II cis-regulatory region sequence-specific DNA binding",
  "gene": "UniProtKB:P24468",
  "term_id": "GO:0000978",
  "gene_name": "COUP transcription factor 2",
  "gene_symbol": "NR2F2"
}